tRNA surveillance [GO:0106354] (biological process) References: PMID:32841241 Sources: GOC:mah Subtypes: TRAMP-dependent tRNA surveillance pathway [GO:0071038], rapid tRNA decay [GO:0180037] Definition: The set of processes involved in identifying and degrading defective or aberrant tRNAs. Relationships: is_a tRNA decay [GO:0016078]; is a type of RNA surveillance [GO:0071025]